serine protease inhibitor complex [GO:0097180] (cellular component) Also known as: serine-type endopeptidase inhibitor complex, serpin complex References: PMID:6323392 Sources: GOC:ans Definition: A heterodimeric protein complex that contains a serine protease inhibitor and a protease; formation of the complex inhibits serine protease activity. Relationships: is a type of protease inhibitor complex [GO:0097179] Subtypes: protein C inhibitor-acrosin complex [GO:0033282], protein C inhibitor-TMPRSS7 complex [GO:0036024], protein C inhibitor-TMPRSS11E complex [GO:0036025], protein C inhibitor-PLAT complex [GO:0036026], protein C inhibitor-PLAU complex [GO:0036027], GO:0036028, protein C inhibitor-KLK3 complex [GO:0036029], protein C inhibitor-plasma kallikrein complex [GO:0036030], protein C inhibitor-coagulation factor V complex [GO:0097181], GO:0097182, protein C inhibitor-coagulation factor XI complex [GO:0097183]